{
  "term_id": "GO:0019369",
  "gene_name": "Calcium-independent phospholipase A2-gamma",
  "gene_symbol": "PNPLA8",
  "term_label": "arachidonate metabolic process",
  "gene": "UniProtKB:Q9NP80"
}